{
  "term_id": "GO:0072487",
  "gene_symbol": "MSL1",
  "term_label": "MSL complex",
  "gene_name": "Male-specific lethal 1 homolog",
  "gene": "UniProtKB:Q68DK7"
}